{
  "term_label": "Unknown molecular function",
  "gene": "UniProtKB:A8MTA8",
  "gene_name": "Protein FAM166B",
  "term_id": "UNKNOWN:0001",
  "gene_symbol": "FAM166B"
}